{
  "term_id": "UNKNOWN:0001",
  "gene": "UniProtKB:Q8IXA5",
  "gene_name": "Sperm acrosome membrane-associated protein 3",
  "gene_symbol": "SPACA3",
  "term_label": "Unknown molecular function"
}